{
  "gene_name": "Tetratricopeptide repeat protein 8",
  "term_label": "BBSome",
  "gene": "UniProtKB:Q8TAM2",
  "term_id": "GO:0034464",
  "gene_symbol": "TTC8"
}